response to glucoside [GO:1904631] (biological process) Definition: Any process that results in a change in state or activity of a cell or an organism (in terms of movement, secretion, enzyme production, gene expression, etc.) as a result of a glucoside stimulus. References: PMID:16842873 Sources: GOC:TermGenie, GO_REF:0000071 Also known as: response to glucosides Relationships: is a type of response to glycoside [GO:1903416] Subtypes: response to etoposide [GO:1902521], GO:1904632